{
  "gene_name": "Phospholipase A and acyltransferase 3",
  "term_id": "GO:0016410",
  "gene_symbol": "PLAAT3",
  "gene": "UniProtKB:P53816",
  "term_label": "N-acyltransferase activity"
}